T=21/pseudo21 icosahedral capsid [GO:0160169] (cellular component) Relationships: is a type of icosahedral viral capsid [GO:0019030] Sources: VZ:833 Definition: The protein coat that surrounds the infective nucleic acid in some virus particles where the subunits (capsomeres) are arranged to form an icosahedron with T=21 or pseudo T=21 symmetry.